O-acetyltransferase activity [GO:0016413] (molecular function) Definition: Catalysis of the transfer of an acetyl group to an oxygen atom on the acceptor molecule. Relationships: is_a O-acyltransferase activity [GO:0008374]; is a type of acetyltransferase activity [GO:0016407] Sources: GOC:ai Subtypes: alcohol O-acetyltransferase activity [GO:0004026], carnitine O-acetyltransferase activity [GO:0004092], choline O-acetyltransferase activity [GO:0004102], homoserine O-acetyltransferase activity [GO:0004414], chloramphenicol O-acetyltransferase activity [GO:0008811], galactoside O-acetyltransferase activity [GO:0008870], maltose O-acetyltransferase activity [GO:0008925], serine O-acetyltransferase activity [GO:0009001], GO:0010327, glycerone-phosphate O-acyltransferase activity [GO:0016287], trichothecene 3-O-acetyltransferase activity [GO:0045462], N-hydroxyarylamine O-acetyltransferase activity [GO:0046990], alkylglycerophosphate 2-O-acetyltransferase activity [GO:0047160], 17-O-deacetylvindoline O-acetyltransferase activity [GO:0047162], salutaridinol 7-O-acetyltransferase activity [GO:0047180], N-acetylneuraminate 4-O-acetyltransferase activity [GO:0047185], N-acetylneuraminate 9-O-acetyltransferase activity [GO:0047186], GO:0047188, GO:0047192, cortisol O-acetyltransferase activity [GO:0047784], monoterpenol O-acetyltransferase activity [GO:0050107], N6-hydroxylysine O-acetyltransferase activity [GO:0050133], GO:0050208, taxadien-5-alpha-ol O-acetyltransferase activity [GO:0050638], 10-hydroxytaxane O-acetyltransferase activity [GO:0050639], 10-deacetylbaccatin III 10-O-acetyltransferase activity [GO:0050643], xylan O-acetyltransferase activity [GO:1990538]